{
  "gene_symbol": "AFG2B",
  "gene": "UniProtKB:Q9BVQ7",
  "term_label": "mitotic spindle disassembly",
  "term_id": "GO:0051228",
  "gene_name": "ATPase family gene 2 protein homolog B"
}